cellular response to xenobiotic stimulus [GO:0071466] (biological process) Also known as: cellular response to drug Regulation: RO_0002211 by regulation of cellular response to drug [GO:2001038]; negatively regulated by GO:2001039; positively regulated by positive regulation of cellular response to drug [GO:2001040] Definition: Any process that results in a change in state or activity of a cell (in terms of movement, secretion, enzyme production, gene expression, etc.) as a result of a stimulus from a xenobiotic, a compound foreign to the organism exposed to it. It may be synthesized by another organism (like ampicilin) or it can be a synthetic chemical. Sources: GOC:krc, GOC:mah Relationships: is a type of response to xenobiotic stimulus [GO:0009410]; is a type of GO:0070887